ectodermal cell fate commitment [GO:0001712] (biological process) Definition: The cell differentiation process that results in commitment of a cell to become part of the ectoderm. Sources: GOC:go_curators, ISBN:0878932437 Also known as: ectoderm cell fate commitment Relationships: is a type of GO:0060795; is part of ectoderm formation [GO:0001705]; is part of ectodermal cell differentiation [GO:0010668]